{
  "term_id": "GO:0071526",
  "term_label": "semaphorin-plexin signaling pathway",
  "gene_name": "Semaphorin-5B",
  "gene_symbol": "SEMA5B",
  "gene": "UniProtKB:Q9P283"
}